{
  "term_id": "GO:0006493",
  "term_label": "protein O-linked glycosylation",
  "gene_name": "Polypeptide N-acetylgalactosaminyltransferase 14",
  "gene_symbol": "GALNT14",
  "gene": "UniProtKB:Q96FL9"
}